{
  "gene": "UniProtKB:O14964",
  "term_id": "GO:0032456",
  "term_label": "endocytic recycling",
  "gene_symbol": "HGS",
  "gene_name": "Hepatocyte growth factor-regulated tyrosine kinase substrate"
}